{
  "term_label": "intermembrane lipid transfer",
  "gene_symbol": "CPTP",
  "term_id": "GO:0120009",
  "gene": "UniProtKB:Q5TA50",
  "gene_name": "Ceramide-1-phosphate transfer protein"
}